{
  "gene_name": "CD81 antigen",
  "term_id": "UNKNOWN:0001",
  "term_label": "Unknown molecular function",
  "gene_symbol": "CD81",
  "gene": "UniProtKB:P60033"
}